structural molecule activity [GO:0005198] (molecular function) Definition: The action of a molecule that contributes to the structural integrity of a complex. Relationships: is a type of molecular_function [GO:0003674] Sources: GOC:mah, GOC:vw Subtypes: structural constituent of ribosome [GO:0003735], structural constituent of cell wall [GO:0005199], structural constituent of cytoskeleton [GO:0005200], GO:0005201, structural constituent of eye lens [GO:0005212], structural constituent of egg chorion [GO:0005213], structural constituent of bone [GO:0008147], GO:0008307, structural constituent of vitelline membrane [GO:0008316], GO:0016490, structural constituent of nuclear pore [GO:0017056], structural constituent of myelin sheath [GO:0019911], GO:0030280, structural constituent of cutaneous appendage [GO:0030281], structural constituent of chromatin [GO:0030527], GO:0039660, structural constituent of cuticle [GO:0042302], structural constituent of carboxysome shell [GO:0043886], structural constituent of albumen [GO:0097099], structural molecule activity conferring elasticity [GO:0097493], GO:0098918, GO:0140073, structural constituent of cytoplasmic lattice [GO:0140094], structural constituent of proteasome [GO:0140756], structural constituent of nuclear lamina [GO:0160123]